{
  "gene_symbol": "RAC3",
  "term_label": "motor neuron axon guidance",
  "gene_name": "Ras-related C3 botulinum toxin substrate 3",
  "term_id": "GO:0008045",
  "gene": "UniProtKB:P60763"
}